flavonoid 3',5'-hydroxylase activity [GO:0033772] (molecular function) Sources: RHEA:55448 Relationships: is a type of GO:0016709 Definition: Catalysis of the reaction: a 3',5'-unsubstituted flavanone + 2 O2 + 2 reduced [NADPH--hemoprotein reductase] = a 3',5'-dihydroxyflavanone + 2 H+ + 2 H2O + 2 oxidized [NADPH--hemoprotein reductase]. Also known as: F3',5'H, F3'5'H, flavanone,NADPH:oxygen oxidoreductase activity